{
  "gene": "UniProtKB:Q659C4",
  "gene_name": "La-related protein 1B",
  "gene_symbol": "LARP1B",
  "term_id": "GO:0010494",
  "term_label": "cytoplasmic stress granule"
}